linoleate 9S-lipoxygenase activity [GO:1990136] (molecular function) Definition: Catalysis of the reaction: linoleate + O2 = (9S,10E,12Z)-9-hydroperoxy-10,12-octadecadienoate. Relationships: is a type of oxidoreductase activity, acting on single donors with incorporation of molecular oxygen, incorporation of two atoms of oxygen [GO:0016702] Sources: GOC:rph, RHEA:30291 Also known as: linoleate:oxygen 9S-oxidoreductase activity, 9-lipoxygenase activity, 9S-lipoxygenase activity, linoleate 9-lipoxygenase activity